{
  "gene": "UniProtKB:Q9UJ83",
  "term_label": "fatty acid alpha-oxidation",
  "gene_symbol": "HACL1",
  "term_id": "GO:0001561",
  "gene_name": "2-hydroxyacyl-CoA lyase 1"
}